positive regulation of transcription regulatory region DNA binding [GO:2000679] (BP) Relationships: is a type of GO:0043388; is a type of regulation of transcription regulatory region DNA binding [GO:2000677]; positively regulates transcription cis-regulatory region binding [GO:0000976] Definition: Any process that activates or increases the frequency, rate or extent of transcription regulatory region DNA binding. Subtypes: positive regulation of core promoter binding [GO:1904798] Sources: GOC:obol